{
  "gene": "UniProtKB:O43281",
  "gene_symbol": "EFS",
  "term_label": "focal adhesion",
  "gene_name": "Embryonal Fyn-associated substrate",
  "term_id": "GO:0005925"
}